purine nucleoside diphosphate biosynthetic process [GO:0009136] (BP) Subtypes: purine ribonucleoside diphosphate biosynthetic process [GO:0009180], GO:0009183 Also known as: purine nucleoside diphosphate anabolism, purine nucleoside diphosphate biosynthesis, purine nucleoside diphosphate formation, purine nucleoside diphosphate synthesis Definition: The chemical reactions and pathways resulting in the formation of purine nucleoside diphosphate, a compound consisting of a purine base linked to a ribose or deoxyribose sugar esterified with diphosphate on the sugar. Sources: GOC:go_curators, ISBN:0198506732 Relationships: is a type of nucleoside diphosphate biosynthetic process [GO:0009133]; is a type of GO:0009135